cellular response to 11-deoxycorticosterone [GO:1903497] (biological process) Definition: Any process that results in a change in state or activity of a cell (in terms of movement, secretion, enzyme production, gene expression, etc.) as a result of a 11-deoxycorticosterone stimulus. Relationships: is a type of cellular response to mineralocorticoid stimulus [GO:0071389]; is a type of cellular response to alcohol [GO:0097306]; is a type of cellular response to ketone [GO:1901655]; is a type of response to 11-deoxycorticosterone [GO:1903496] References: PMID:3585228 Sources: GOC:TermGenie, GOC:mr, GO_REF:0000071